{
  "gene_name": "VIP peptides",
  "term_id": "GO:0005184",
  "gene_symbol": "VIP",
  "gene": "UniProtKB:P01282",
  "term_label": "neuropeptide hormone activity"
}